{
  "gene": "UniProtKB:Q9NZQ7",
  "gene_name": "Programmed cell death 1 ligand 1",
  "gene_symbol": "CD274",
  "term_id": "GO:0009897",
  "term_label": "external side of plasma membrane"
}